{
  "term_label": "tricarboxylic acid cycle",
  "gene_name": "Malate dehydrogenase, mitochondrial",
  "gene_symbol": "MDH2",
  "gene": "UniProtKB:P40926",
  "term_id": "GO:0006099"
}